{
  "gene_symbol": "RMDN2",
  "term_id": "UNKNOWN:0002",
  "term_label": "Unknown biological process",
  "gene": "UniProtKB:Q96LZ7",
  "gene_name": "Regulator of microtubule dynamics protein 2"
}